tetrachloroethene reductive dehalogenase activity [GO:0050629] (molecular function) Definition: Catalysis of the reaction: trichloroethene + chloride + acceptor = tetrachloroethene + reduced acceptor. The reaction occurs in the reverse direction. Sources: RHEA:20353 Also known as: acceptor:trichloroethene oxidoreductase (chlorinating), tetrachloroethene reductase activity Relationships: is_a oxidoreductase activity, acting on X-H and Y-H to form an X-Y bond [GO:0046992]